{
  "gene_name": "Protein FAM43B",
  "gene": "UniProtKB:Q6ZT52",
  "gene_symbol": "FAM43B",
  "term_id": "UNKNOWN:0001",
  "term_label": "Unknown molecular function"
}